L-leucine transmembrane transporter activity [GO:0015190] (molecular function) Relationships: is a type of neutral L-amino acid transmembrane transporter activity [GO:0015175]; is a type of L-amino acid transmembrane transporter activity [GO:0015179]; is a type of branched-chain amino acid transmembrane transporter activity [GO:0015658] Definition: Enables the transfer of L-leucine from one side of a membrane to the other. L-leucine is 2-amino-4-methylpentanoic acid. Sources: GOC:ai, GOC:mtg_transport, ISBN:0815340729 Also known as: L-leucine transporter activity, leucine/isoleucine/valine porter activity, leucine/valine/isoleucine permease activity